tertiary alcohol metabolic process [GO:1902644] (biological process) Definition: The chemical reactions and pathways involving tertiary alcohol. References: PMID:11288200 Sources: GOC:TermGenie, GOC:mengo_curators, GO_REF:0000068 Also known as: tertiary alcohol metabolism Relationships: is a type of GO:0006066 Subtypes: abscisic acid metabolic process [GO:0009687], cortisol metabolic process [GO:0034650], doxorubicin metabolic process [GO:0044598], rhodopsin catabolic process [GO:0046155], GO:1900553, tetracenomycin C catabolic process [GO:1901105], GO:1902049, cis-abienol catabolic process [GO:1902245], GO:1902645